{
  "gene_name": "N-chimaerin",
  "gene_symbol": "CHN1",
  "term_id": "UNKNOWN:0003",
  "term_label": "Unknown cellular component",
  "gene": "UniProtKB:P15882"
}